meiotic spindle elongation [GO:0051232] (biological process) Sources: GOC:ai Also known as: spindle elongation during meiosis Relationships: is a type of spindle elongation [GO:0051231]; is a type of meiotic cell cycle process [GO:1903046]; is part of meiotic spindle organization [GO:0000212]; is part of meiotic chromosome segregation [GO:0045132] Regulation: regulated by regulation of meiotic spindle elongation [GO:1902119]; RO_0002212 by GO:1902120 Definition: The lengthening of the distance between poles of the spindle during a meiotic cell cycle.